{
  "term_label": "basement membrane",
  "gene_name": "Laminin subunit gamma-1",
  "gene": "UniProtKB:P11047",
  "gene_symbol": "LAMC1",
  "term_id": "GO:0005604"
}